{
  "gene_symbol": "ATXN7L3",
  "gene_name": "Ataxin-7-like protein 3",
  "term_id": "GO:0045893",
  "gene": "UniProtKB:Q14CW9",
  "term_label": "positive regulation of DNA-templated transcription"
}